{
  "term_id": "GO:0060271",
  "gene": "UniProtKB:Q9UPM9",
  "term_label": "cilium assembly",
  "gene_name": "B9 domain-containing protein 1",
  "gene_symbol": "B9D1"
}